ERCC4-ERCC1 complex [GO:0070522] (cellular component) Relationships: is a type of GO:0000109 Definition: A heterodimeric nucleotide-excision repair complex that has endonuclease activity specific for bubble structures characteristic of certain DNA lesions. The subunits are known as XPF/ERCC4 and ERCC1 in mammals, and Rad1p and Rad10p in S. cerevisiae. Also known as: Rad1-Rad10 complex, XPF-ERCC1 complex Note: Note that process and function information are included in the term and definition for the purpose of describing and distinguishing the complex. References: PMID:14734547